protochlorophyllide reductase activity [GO:0016630] (molecular function) Also known as: NADPH-protochlorophyllide oxidoreductase activity, NADPH-protochlorophyllide reductase activity, NADPH2-protochlorophyllide oxidoreductase activity, chlorophyllide-a:NADP+ 7,8-oxidoreductase activity, protochlorophyllide oxidoreductase activity, protochlorophyllide photooxidoreductase activity Sources: EC:1.3.1.33 Definition: Catalysis of the reaction: chlorophyllide a + NADP+ = protochlorophyllide + NADPH + H+. Relationships: is a type of oxidoreductase activity, acting on the CH-CH group of donors, NAD or NADP as acceptor [GO:0016628]